positive regulation of cuticle pigmentation [GO:0048081] (biological process) Also known as: up regulation of cuticle pigmentation, up-regulation of cuticle pigmentation, upregulation of cuticle pigmentation, activation of cuticle pigmentation, stimulation of cuticle pigmentation Relationships: is a type of regulation of cuticle pigmentation [GO:0048079]; is a type of positive regulation of developmental pigmentation [GO:0048087]; is a type of GO:0051094; is a type of positive regulation of multicellular organismal process [GO:0051240]; positively regulates GO:0048067 Definition: Any process that activates or increases the frequency, rate or extent of establishment of a pattern of pigment in the cuticle of an organism. Subtypes: positive regulation of adult chitin-containing cuticle pigmentation [GO:0048084] Sources: GOC:jid